amino acid export across plasma membrane [GO:0032973] (biological process) Regulation: regulated by regulation of amino acid export [GO:0080143] Also known as: amino acid export, amino acid transmembrane export, amino acid efflux Sources: GOC:jl Relationships: is a type of amino acid transmembrane transport [GO:0003333]; is a type of export across plasma membrane [GO:0140115] Definition: The directed movement of amino acids from inside of a cell, across the plasma membrane and into the extracellular region. Subtypes: cysteine export across plasma membrane [GO:0033228], GO:0140406